{
  "gene_name": "Protein SERAC1",
  "term_label": "Unknown molecular function",
  "term_id": "UNKNOWN:0001",
  "gene": "UniProtKB:Q96JX3",
  "gene_symbol": "SERAC1"
}